{
  "term_label": "Unknown molecular function",
  "term_id": "UNKNOWN:0001",
  "gene_symbol": "MFAP1",
  "gene": "UniProtKB:P55081",
  "gene_name": "Microfibrillar-associated protein 1"
}